apoptotic mitochondrial changes [GO:0008637] (biological process) Relationships: is a type of GO:0007005; is part of apoptotic process [GO:0006915] Note: This term was created to reflect the fundamental role of the mitochondrial compartment in apoptosis. Most processes under this node occur during the signaling phase of apoptosis, but e.g. GO:0043653 'mitochondrial fragmentation involved in apoptotic process' cannot be confidently placed under the signaling phase. For this reason, the parent term GO:0008637 'apoptotic mitochondrial changes' is not linked to the signaling or execution phase specifically, but its descendants are when current knowledge allows for it. Definition: The morphological and physiological alterations undergone by mitochondria during apoptosis. Subtypes: GO:0001836, release of matrix enzymes from mitochondria [GO:0032976], mitochondrial fragmentation involved in apoptotic process [GO:0043653], regulation of mitochondrial membrane permeability involved in apoptotic process [GO:1902108] Sources: GOC:mah, GOC:mtg_apoptosis